BAX complex [GO:0097144] (cellular component) Definition: An oligomeric protein complex consisting of BAX, a member of the Bcl-2 family of anti- and proapoptotic regulators. References: PMID:14634621 Sources: GOC:so Relationships: is a type of Bcl-2 family protein complex [GO:0097136]